pyrophosphate-dependent phosphofructokinase complex [GO:0010316] (CC) Also known as: PFK complex Relationships: is a type of catalytic complex [GO:1902494] Definition: Heterodimeric complex that catalyzes the pyrophosphate-dependent phosphorylation of D-fructose 6-phosphate into D-fructose 1,6-bisphosphate. References: PMID:2170409